neuron projection [GO:0043005] (cellular component) Subtypes: axon [GO:0030424], dendrite [GO:0030425], stereocilium [GO:0032420], neuron spine [GO:0044309], rod spherule [GO:0044317], kinocilium [GO:0060091], cell body fiber [GO:0070852], dendritic tree [GO:0097447], Lewy neurite [GO:0097462], GO:0097463, GO:0097733, telodendria [GO:0120208], dendritic filopodium [GO:1902737], growth cone lamellipodium [GO:1990761], proximal neuron projection [GO:1990769], GO:1990812, accessory outer segment [GO:1990906] References: PMID:3077060 Sources: GOC:jl Relationships: is a type of plasma membrane bounded cell projection [GO:0120025] Also known as: neuron process, neuron protrusion, neuronal cell projection, neurite, nerve fiber Definition: A prolongation or process extending from a nerve cell, e.g. an axon or dendrite.